4-hydroxyproline epimerase activity [GO:0047580] (molecular function) Sources: EC:5.1.1.8, RHEA:21152 Definition: Catalysis of the reaction: trans-4-hydroxy-L-proline = cis-4-hydroxy-D-proline. Also known as: 4-hydroxyproline 2-epimerase activity, L-hydroxyproline epimerase activity, hydroxyproline 2-epimerase activity, hydroxyproline epimerase activity Relationships: is a type of amino-acid racemase activity [GO:0047661]